{
  "gene": "UniProtKB:Q9NQI0",
  "term_id": "GO:0043186",
  "gene_name": "Probable ATP-dependent RNA helicase DDX4",
  "gene_symbol": "DDX4",
  "term_label": "P granule"
}